mitochondrial ribosomal large subunit rRNA binding [GO:1990400] (molecular function) Relationships: is a type of large ribosomal subunit rRNA binding [GO:0070180] Also known as: mitochondrial LSU rRNA binding, 21S rRNA binding References: PMID:24206665 Note: In S. cerevisiae, this is the mitochondrial 21S rRNA Definition: Binding to a mitochondrial large ribosomal subunit RNA (LSU rRNA).